regulation of tube length, open tracheal system [GO:0035159] (biological process) Also known as: regulation of tracheal tube length, tracheal tube elongation Relationships: is a type of regulation of tube size, open tracheal system [GO:0035151] Definition: Ensuring that a tube in an open tracheal system is of the correct length. Sources: GOC:bf, GOC:mtg_sensu